carbon-nitrogen lyase activity [GO:0016840] (molecular function) Sources: EC:4.3.-.- Relationships: is a type of lyase activity [GO:0016829] Definition: Catalysis of the release of ammonia or one of its derivatives, with the formation of a double bond or ring. Enzymes with this activity may catalyze the actual elimination of the ammonia, amine or amide, e.g. CH-CH(-NH-R) = C=CH- + NH2-R. Others, however, catalyze elimination of another component, e.g. water, which is followed by spontaneous reactions that lead to breakage of the C-N bond, e.g. L-serine ammonia-lyase (EC:4.3.1.17), so that the overall reaction is C(-OH)-CH(-NH2) = CH2-CO- + NH3, i.e. an elimination with rearrangement. The sub-subclasses of EC:4.3 are the ammonia-lyases (EC:4.3.1), lyases acting on amides, amidines, etc. (EC:4.3.2), the amine-lyases (EC:4.3.3), and other carbon-nitrogen lyases (EC:4.3.99). Subtypes: GO:0008824, ammonia-lyase activity [GO:0016841], GO:0016842, amine-lyase activity [GO:0016843], choline trimethylamine lyase activity [GO:0120525] Also known as: other carbon-nitrogen lyase activity